regulation of telomere maintenance via telomere lengthening [GO:1904356] (biological process) Subtypes: GO:0032210, negative regulation of telomere maintenance via telomere lengthening [GO:1904357], positive regulation of telomere maintenance via telomere lengthening [GO:1904358] References: PMID:23959892 Sources: GOC:BHF, GOC:BHF_telomere, GOC:TermGenie, GOC:nc, GO_REF:0000058 Relationships: is a type of regulation of telomere maintenance [GO:0032204]; regulates telomere maintenance via telomere lengthening [GO:0010833] Definition: Any process that modulates the frequency, rate or extent of telomere maintenance via telomere lengthening.